{
  "gene_name": "F-box only protein 24",
  "term_label": "Unknown biological process",
  "term_id": "UNKNOWN:0002",
  "gene_symbol": "FBXO24",
  "gene": "UniProtKB:O75426"
}